positive regulation of hyaluronan biosynthetic process [GO:1900127] (BP) Definition: Any process that activates or increases the frequency, rate or extent of hyaluronan biosynthetic process. Sources: GOC:TermGenie, GOC:yaf Relationships: is a type of positive regulation of macromolecule biosynthetic process [GO:0010557]; is a type of positive regulation of carbohydrate metabolic process [GO:0045913]; is a type of regulation of hyaluronan biosynthetic process [GO:1900125]; positively regulates hyaluronan biosynthetic process [GO:0030213] Also known as: activation of hyaluronan anabolism, activation of hyaluronan biosynthesis, activation of hyaluronan formation, activation of hyaluronan synthesis, positive regulation of hyaluronan anabolism, positive regulation of hyaluronan biosynthesis, positive regulation of hyaluronan formation, positive regulation of hyaluronan synthesis, up regulation of hyaluronan anabolism, up regulation of hyaluronan biosynthesis, up regulation of hyaluronan biosynthetic process, up regulation of hyaluronan formation, up regulation of hyaluronan synthesis, up-regulation of hyaluronan anabolism, up-regulation of hyaluronan biosynthesis, up-regulation of hyaluronan biosynthetic process, up-regulation of hyaluronan formation, up-regulation of hyaluronan synthesis, upregulation of hyaluronan anabolism, upregulation of hyaluronan biosynthesis, upregulation of hyaluronan biosynthetic process, upregulation of hyaluronan formation, upregulation of hyaluronan synthesis, activation of hyaluronan biosynthetic process